{
  "term_label": "cytoplasm",
  "term_id": "GO:0005737",
  "gene_symbol": "CDC16",
  "gene_name": "Cell division cycle protein 16 homolog",
  "gene": "UniProtKB:Q13042"
}